{
  "gene": "UniProtKB:P23763",
  "gene_symbol": "VAMP1",
  "term_label": "vesicle fusion",
  "term_id": "GO:0006906",
  "gene_name": "Vesicle-associated membrane protein 1"
}